{
  "gene": "UniProtKB:Q9UJ96",
  "term_id": "GO:0008076",
  "term_label": "voltage-gated potassium channel complex",
  "gene_name": "Potassium voltage-gated channel subfamily G member 2",
  "gene_symbol": "KCNG2"
}